{
  "term_id": "GO:0006886",
  "gene": "UniProtKB:Q8WU76",
  "gene_name": "Sec1 family domain-containing protein 2",
  "term_label": "intracellular protein transport",
  "gene_symbol": "SCFD2"
}